2-oxoglutarate oxygenase/decarboxylase (ethylene-forming) activity [GO:0102276] (molecular function) Relationships: is a type of oxidoreductase activity, acting on single donors with incorporation of molecular oxygen, incorporation of one atom of oxygen (internal monooxygenases or internal mixed function oxidases) [GO:0016703] Sources: EC:1.13.12.19, GOC:pz Definition: Catalysis of the reaction: 2-oxoglutarate(2-) + O2 + 2 H+ = ethene + 3 carbon dioxide + H2O.